triglyceride binding [GO:0017129] (molecular function) Relationships: is a type of lipid binding [GO:0008289] Sources: GOC:jl, ISBN:0198506732 Definition: Binding to a triester of glycerol. Also known as: triacylglycerol binding